{
  "term_label": "transmembrane signaling receptor activity",
  "gene_symbol": "KREMEN1",
  "gene_name": "Kremen protein 1",
  "term_id": "GO:0004888",
  "gene": "UniProtKB:Q96MU8"
}